oligodendrocyte development [GO:0014003] (biological process) Definition: The process aimed at the progression of an oligodendrocyte over time, from initial commitment of the cell to a specific fate, to the fully functional differentiated cell. An oligodendrocyte is a type of glial cell involved in myelinating the axons in the central nervous system. Relationships: is a type of glial cell development [GO:0021782]; is part of oligodendrocyte differentiation [GO:0048709] Also known as: oligodendrocyte cell development Sources: GOC:dgh, GOC:ef